positive regulation of chromosome segregation [GO:0051984] (biological process) Definition: Any process that activates or increases the frequency, rate or extent of chromosome segregation, the process in which genetic material, in the form of chromosomes, is organized and then physically separated and apportioned to two or more sets. Subtypes: positive regulation of attachment of spindle microtubules to kinetochore [GO:0051987], GO:0062033 Sources: GOC:ai Relationships: is a type of regulation of chromosome segregation [GO:0051983]; is a type of GO:0090068; positively regulates chromosome segregation [GO:0007059] Also known as: up regulation of chromosome segregation, up-regulation of chromosome segregation, upregulation of chromosome segregation, activation of chromosome segregation, stimulation of chromosome segregation